{
  "gene_symbol": "PPM1G",
  "term_id": "GO:0007165",
  "gene_name": "Protein phosphatase 1G",
  "term_label": "signal transduction",
  "gene": "UniProtKB:O15355"
}